{
  "term_label": "membrane",
  "term_id": "GO:0016020",
  "gene": "UniProtKB:Q86WI0",
  "gene_symbol": "LHFPL1",
  "gene_name": "LHFPL tetraspan subfamily member 1 protein"
}